positive regulation of miRNA-mediated gene silencing [GO:2000637] (biological process) Sources: GOC:dph Also known as: positive regulation of gene silencing by miRNA, positive regulation of microRNA-mediated gene silencing, positive regulation of gene silencing by microRNA Definition: A process that activates or increases the frequency, rate or extent of gene silencing by a microRNA (miRNA). Relationships: is a type of regulation of miRNA-mediated gene silencing [GO:0060964]; is a type of positive regulation of post-transcriptional gene silencing by RNA [GO:1900370]; positively regulates GO:0035195 Subtypes: GO:1903800